symbiont-mediated perturbation of host actin cytoskeleton via actin crosslinking [GO:0141031] (BP) References: PMID:14512630, PMID:22814176 Definition: The process in which an organism effects a change that impairs the structure or function of the host actin cytoskeleton by actin crosslinking the host actin filaments. The host is defined as the larger of the organisms involved in a symbiotic interaction. Relationships: is a type of symbiont-mediated perturbation of host actin cytoskeleton [GO:0141027] Also known as: perturbation by symbiont of host actin cytoskeleton via actin crosslinking